{
  "gene": "UniProtKB:Q8TCD1",
  "term_id": "UNKNOWN:0001",
  "gene_symbol": "C18orf32",
  "term_label": "Unknown molecular function",
  "gene_name": "UPF0729 protein C18orf32"
}